{
  "gene": "UniProtKB:Q00613",
  "term_id": "UNKNOWN:0002",
  "term_label": "Unknown biological process",
  "gene_symbol": "HSF1",
  "gene_name": "Heat shock factor protein 1"
}